{
  "gene": "UniProtKB:Q05923",
  "gene_name": "Dual specificity protein phosphatase 2",
  "term_id": "GO:0004721",
  "term_label": "phosphoprotein phosphatase activity",
  "gene_symbol": "DUSP2"
}